{
  "gene": "UniProtKB:O75908",
  "gene_symbol": "SOAT2",
  "term_id": "GO:0034736",
  "gene_name": "Sterol O-acyltransferase 2",
  "term_label": "cholesterol O-acyltransferase activity"
}